interleukin-3 production [GO:0032632] (biological process) Sources: GOC:mah Also known as: IL-3 production, interleukin-3 biosynthetic process, interleukin-3 secretion Definition: The appearance of interleukin-3 due to biosynthesis or secretion following a cellular stimulus, resulting in an increase in its intracellular or extracellular levels. Regulation: regulated by regulation of interleukin-3 production [GO:0032672]; negatively regulated by negative regulation of interleukin-3 production [GO:0032712]; positively regulated by positive regulation of interleukin-3 production [GO:0032752] Relationships: is a type of GO:0001816